establishment of mitochondrion localization [GO:0051654] (biological process) Relationships: is a type of GO:0051646; is a type of establishment of organelle localization [GO:0051656] Also known as: establishment of mitochondria localization, establishment of mitochondrion localisation, mitochondria positioning, mitochondrial migration, mitochondrion positioning Definition: The directed movement of the mitochondrion to a specific location. Subtypes: mitochondrion migration along actin filament [GO:0034642], establishment of mitochondrion localization, microtubule-mediated [GO:0034643], GO:0160040 Sources: GOC:ai